{
  "term_label": "protein disulfide isomerase activity",
  "gene_symbol": "P4HB",
  "gene_name": "Protein disulfide-isomerase",
  "gene": "UniProtKB:P07237",
  "term_id": "GO:0003756"
}